{
  "term_id": "GO:0098967",
  "term_label": "exocytic insertion of neurotransmitter receptor to postsynaptic membrane",
  "gene": "UniProtKB:Q13277",
  "gene_name": "Syntaxin-3",
  "gene_symbol": "STX3"
}